{
  "gene_symbol": "PLPP5",
  "term_id": "GO:0046839",
  "gene_name": "Phospholipid phosphatase 5",
  "term_label": "phospholipid dephosphorylation",
  "gene": "UniProtKB:Q8NEB5"
}